adult somatic muscle development [GO:0007527] (biological process) Definition: The process whose specific outcome is the progression of the adult somatic muscle over time, from its formation to the mature structure. Sources: GOC:jid Regulation: RO_0002211 by regulation of adult somatic muscle development [GO:0062226]; positively regulated by positive regulation of adult somatic muscle development [GO:0062227]; negatively regulated by negative regulation of adult somatic muscle development [GO:0062228] Relationships: is a type of somatic muscle development [GO:0007525]